{
  "gene_symbol": "MERTK",
  "gene": "UniProtKB:Q12866",
  "term_label": "transmembrane receptor protein tyrosine kinase activity",
  "gene_name": "Tyrosine-protein kinase Mer",
  "term_id": "GO:0004714"
}